{
  "gene": "UniProtKB:A0A1B0GX31",
  "gene_name": "T cell receptor beta variable 7-6",
  "term_label": "plasma membrane",
  "term_id": "GO:0005886",
  "gene_symbol": "TRBV7-6"
}